{
  "gene_symbol": "TGFBR1",
  "term_id": "GO:0048185",
  "gene": "UniProtKB:P36897",
  "term_label": "activin binding",
  "gene_name": "TGF-beta receptor type-1"
}